{
  "gene": "UniProtKB:Q96R05",
  "term_label": "fatty acid binding",
  "gene_symbol": "RBP7",
  "gene_name": "Retinoid-binding protein 7",
  "term_id": "GO:0005504"
}